metanephric cap mesenchymal cell proliferation involved in metanephros development [GO:0090094] (biological process) Regulation: regulated by GO:0090095; positively regulated by positive regulation of metanephric cap mesenchymal cell proliferation [GO:0090096] References: PMID:19161241 Sources: GOC:dph, GOC:tb, GOC:yaf Definition: The multiplication or reproduction of metanephric cap mesenchymal cells, resulting in the expansion of the cell population. A metanephric cap mesenchymal cell is a mesenchymal cell that has condensed with other mesenchymal cells surrounding the ureteric bud tip. Relationships: is a type of mesenchymal cell proliferation [GO:0010463]; is a type of cell proliferation involved in metanephros development [GO:0072203]; is part of metanephric cap morphogenesis [GO:0072186]